negative regulation of apoptotic DNA fragmentation [GO:1902511] (biological process) Also known as: down regulation of DNA catabolic process during apoptosis, down regulation of DNA catabolism during apoptosis, down regulation of DNA fragmentation involved in apoptotic nuclear change, down regulation of apoptotic DNA fragmentation, down regulation of endonucleolytic DNA catabolic process involved in apoptosis, down-regulation of DNA catabolic process during apoptosis, down-regulation of DNA catabolism during apoptosis, down-regulation of DNA fragmentation involved in apoptotic nuclear change, down-regulation of apoptotic DNA fragmentation, down-regulation of endonucleolytic DNA catabolic process involved in apoptosis, downregulation of DNA catabolic process during apoptosis, downregulation of DNA catabolism during apoptosis, downregulation of DNA fragmentation involved in apoptotic nuclear change, downregulation of apoptotic DNA fragmentation, downregulation of endonucleolytic DNA catabolic process involved in apoptosis, negative regulation of DNA catabolic process during apoptosis, negative regulation of DNA catabolism during apoptosis, negative regulation of DNA fragmentation involved in apoptotic nuclear change, negative regulation of endonucleolytic DNA catabolic process involved in apoptosis, inhibition of DNA catabolic process during apoptosis, inhibition of DNA catabolism during apoptosis, inhibition of DNA fragmentation involved in apoptotic nuclear change, inhibition of apoptotic DNA fragmentation, inhibition of endonucleolytic DNA catabolic process involved in apoptosis Relationships: is a type of regulation of apoptotic DNA fragmentation [GO:1902510]; is a type of GO:1903625; negatively regulates GO:0006309 Definition: Any process that stops, prevents or reduces the frequency, rate or extent of apoptotic DNA fragmentation. References: PMID:15572351 Sources: GOC:TermGenie, GOC:hjd